pteridine reductase activity [GO:0047040] (molecular function) Relationships: is_a oxidoreductase activity, acting on the CH-NH group of donors, NAD or NADP as acceptor [GO:0016646] Definition: Catalysis of the reaction: 5,6,7,8-tetrahydrobiopterin + 2 NADP+ = biopterin + 2 H+ + 2 NADPH. Sources: EC:1.5.1.33, RHEA:19509 Also known as: pteridine reductase 1 activity, ptr1 activity, 5,6,7,8-tetrahydrobiopterin:NADP+ oxidoreductase activity, PTR1, dihydrobiopterin reduction